{
  "term_id": "GO:0005968",
  "gene_symbol": "CHM",
  "gene": "UniProtKB:P24386",
  "term_label": "Rab-protein geranylgeranyltransferase complex",
  "gene_name": "Rab proteins geranylgeranyltransferase component A 1"
}